N6-methyl-lysine oxidase activity [GO:0050134] (molecular function) Also known as: 6-N-methyl-L-lysine:oxygen oxidoreductase (demethylating), N(6)-methyllysine oxidase activity, N6-methyl-L-lysine:oxygen oxidoreductase (demethylating), N6-methyllysine oxidase activity, epsilon-N-methyllysine demethylase activity, epsilon-alkyl-L-lysine:oxygen oxidoreductase activity, epsilon-alkyllysinase activity Relationships: is a type of oxidoreductase activity, acting on the CH-NH group of donors, oxygen as acceptor [GO:0016647] Sources: EC:1.5.3.4, RHEA:23200 Definition: Catalysis of the reaction: N(6)-methyl-L-lysine + H2O + O2 = L-lysine + formaldehyde + H2O2.